{
  "gene": "UniProtKB:Q9H8H2",
  "gene_name": "Probable ATP-dependent RNA helicase DDX31",
  "gene_symbol": "DDX31",
  "term_label": "nucleus",
  "term_id": "GO:0005634"
}